{
  "gene": "UniProtKB:Q96IF1",
  "term_label": "cytoskeleton organization",
  "gene_name": "LIM domain-containing protein ajuba",
  "term_id": "GO:0007010",
  "gene_symbol": "AJUBA"
}